acute-phase response [GO:0006953] (biological process) Sources: ISBN:0198506732 Relationships: is a type of acute inflammatory response [GO:0002526] Definition: An acute inflammatory response that involves non-antibody proteins whose concentrations in the plasma increase in response to infection or injury of homeothermic animals. Subtypes: fever generation [GO:0001660]